{
  "gene": "UniProtKB:P35908",
  "gene_symbol": "KRT2",
  "term_id": "GO:0030280",
  "term_label": "structural constituent of skin epidermis",
  "gene_name": "Keratin, type II cytoskeletal 2 epidermal"
}